{
  "term_id": "GO:1990756",
  "gene_name": "PRAME family member 19",
  "gene_symbol": "PRAMEF19",
  "gene": "UniProtKB:Q5SWL8",
  "term_label": "ubiquitin-like ligase-substrate adaptor activity"
}